{
  "gene_symbol": "CDK5RAP1",
  "gene": "UniProtKB:Q96SZ6",
  "term_label": "cytosol",
  "term_id": "GO:0005829",
  "gene_name": "Mitochondrial tRNA methylthiotransferase CDK5RAP1"
}